beta-catenin-TCF7L2 complex [GO:0070369] (CC) Also known as: beta-catenin-TCF4 complex Relationships: is a type of GO:0071664; is a type of GO:1990907 References: PMID:9065401, PMID:9065402 Sources: GOC:BHF, GOC:rl Definition: A protein complex that contains beta-catenin and TCF7L2 (TCF4), binds to the TCF DNA motif within a promoter element, and is involved in the regulation of WNT target gene transcription.